gamma-glutamylhistamine synthase activity [GO:0047914] (MF) Also known as: g-glutamylhistamine synthase activity, L-glutamate:histamine ligase activity, gamma-GHA synthetase activity, gamma-glutaminylhistamine synthetase activity Definition: Catalysis of the reaction: histamine + L-glutamate + ATP = N(alpha)-gamma-L-glutamylhistamine + products of ATP breakdown. Relationships: is a type of GO:0016881 Sources: EC:6.3.2.18, MetaCyc:GAMMA-GLUTAMYLHISTAMINE-SYNTHASE-RXN